{
  "term_id": "GO:0031297",
  "gene": "UniProtKB:A8MT69",
  "gene_symbol": "CENPX",
  "term_label": "replication fork processing",
  "gene_name": "Centromere protein X"
}